{
  "gene": "UniProtKB:Q8N3U1",
  "gene_symbol": "Q8N3U1",
  "term_id": "UNKNOWN:0001",
  "term_label": "Unknown molecular function",
  "gene_name": "Putative uncharacterized protein LOC400692"
}